glycolipid transport [GO:0046836] (biological process) Relationships: is a type of lipid transport [GO:0006869]; is_a carbohydrate derivative transport [GO:1901264] Definition: The directed movement of glycolipids, compounds containing (usually) 1-4 linked monosaccharide residues joined by a glycosyl linkage to a lipid, into, out of or within a cell, or between cells, by means of some agent such as a transporter or pore. Subtypes: glycolipid translocation [GO:0034203], ganglioside GM1 transport to membrane [GO:1905572] Sources: GOC:ai